{
  "gene_name": "Small ribosomal subunit protein eS27",
  "gene": "UniProtKB:P42677",
  "gene_symbol": "RPS27",
  "term_label": "structural constituent of ribosome",
  "term_id": "GO:0003735"
}